{
  "gene_symbol": "RESF1",
  "gene_name": "Retroelement silencing factor 1",
  "term_label": "nucleus",
  "term_id": "GO:0005634",
  "gene": "UniProtKB:Q9HCM1"
}